regulation of N-terminal protein palmitoylation [GO:0060254] (biological process) Definition: Any process that modulates the rate frequency or extent of the covalent attachment of a palmitoyl group to the N-terminal amino acid residue of a protein. Subtypes: negative regulation of N-terminal protein palmitoylation [GO:0060262] Sources: GOC:dph, GOC:tb Relationships: is a type of regulation of protein lipidation [GO:1903059]; regulates N-terminal protein palmitoylation [GO:0006500]